{
  "gene": "UniProtKB:Q14146",
  "term_label": "ribosome biogenesis",
  "gene_symbol": "URB2",
  "term_id": "GO:0042254",
  "gene_name": "Unhealthy ribosome biogenesis protein 2 homolog"
}